histone H2AK5ac reader activity [GO:0140130] (molecular function) References: PMID:18469222 Note: Note that the residue position corresponds to the canonical human H2A2A histone (UniProtKB:Q6FI13); this residue is conserved across all eukaryotes. Corresponds to H2AK4 in yeast and in flies. Residue 1 is the first residue following removal of the initiating Methionine (Met). Note that each histone is encoded by multiple genes, and sequences may vary across different genes within an organism. Definition: A histone reader that recognizes a histone H2A acetylated at lysine 5. Relationships: is a type of GO:0140054